{
  "gene_symbol": "KRTAP2-1",
  "term_id": "UNKNOWN:0002",
  "term_label": "Unknown biological process",
  "gene": "UniProtKB:Q9BYU5",
  "gene_name": "Keratin-associated protein 2-1"
}